{
  "gene_symbol": "C1QL4",
  "gene": "UniProtKB:Q86Z23",
  "gene_name": "Complement C1q-like protein 4",
  "term_label": "Unknown molecular function",
  "term_id": "UNKNOWN:0001"
}